{
  "gene": "UniProtKB:P21953",
  "gene_name": "2-oxoisovalerate dehydrogenase subunit beta, mitochondrial",
  "term_label": "response to nutrient",
  "gene_symbol": "BCKDHB",
  "term_id": "GO:0007584"
}